imaginal disc-derived wing vein specification [GO:0007474] (biological process) Regulation: regulated by regulation of imaginal disc-derived wing vein specification [GO:0110107]; positively regulated by positive regulation of imaginal disc-derived wing vein specification [GO:0110108]; negatively regulated by negative regulation of imaginal disc-derived wing vein specification [GO:0110109] Sources: GOC:dph, GOC:isa_complete, GOC:mtg_sensu Also known as: wing vein specification Definition: The regionalization process in which the area of a imaginal disc-derived wing that will form a wing vein is specified. Relationships: is_a regionalization [GO:0003002]; is part of imaginal disc-derived wing morphogenesis [GO:0007476]